{
  "gene": "UniProtKB:P62273",
  "gene_symbol": "RPS29",
  "gene_name": "Small ribosomal subunit protein uS14",
  "term_id": "GO:0022627",
  "term_label": "cytosolic small ribosomal subunit"
}